{
  "gene": "UniProtKB:P55042",
  "term_label": "plasma membrane",
  "gene_name": "GTP-binding protein RAD",
  "gene_symbol": "RRAD",
  "term_id": "GO:0005886"
}